{
  "term_id": "GO:0020037",
  "gene_symbol": "CYP46A1",
  "term_label": "heme binding",
  "gene_name": "Cholesterol 24-hydroxylase",
  "gene": "UniProtKB:Q9Y6A2"
}